positive regulation of interleukin-4-dependent isotype switching to IgE isotypes [GO:2000572] (biological process) Also known as: positive regulation of IL-4-dependent isotype switching to IgE isotypes Sources: GOC:obol Definition: Any process that activates or increases the frequency, rate or extent of interleukin-4-dependent isotype switching to IgE isotypes. Relationships: is a type of positive regulation of isotype switching to IgE isotypes [GO:0048295]; is a type of regulation of interleukin-4-dependent isotype switching to IgE isotypes [GO:2000571]; RO_0002213 interleukin-4-dependent isotype switching to IgE isotypes [GO:0035708]